{
  "term_id": "GO:0005615",
  "gene_symbol": "IFNA5",
  "gene_name": "Interferon alpha-5",
  "term_label": "extracellular space",
  "gene": "UniProtKB:P01569"
}